{
  "term_label": "L-tryptophan catabolic process to kynurenine",
  "gene": "UniProtKB:Q6ZQW0",
  "term_id": "GO:0019441",
  "gene_symbol": "IDO2",
  "gene_name": "Indoleamine 2,3-dioxygenase 2"
}